{
  "term_id": "GO:0006044",
  "gene": "UniProtKB:Q8NCG5",
  "gene_symbol": "CHST4",
  "term_label": "N-acetylglucosamine metabolic process",
  "gene_name": "Carbohydrate sulfotransferase 4"
}